{
  "term_label": "Unknown biological process",
  "gene_name": "Putative ciliary rootlet coiled-coil protein-like 1 protein",
  "gene": "UniProtKB:Q86T23",
  "term_id": "UNKNOWN:0002",
  "gene_symbol": "CROCCP2"
}